regulation of erythrocyte enucleation [GO:0061930] (biological process) Definition: Any process that modulates the frequency, rate or extent of erythrocyte enucleation. Relationships: is a type of regulation of cellular component organization [GO:0051128]; is a type of GO:1903429; regulates erythrocyte enucleation [GO:0043131] Subtypes: positive regulation of erythrocyte enucleation [GO:0061931], GO:0061932 References: PMID:25241935